{
  "term_id": "GO:0005109",
  "gene": "UniProtKB:Q9H1J5",
  "term_label": "frizzled binding",
  "gene_name": "Protein Wnt-8a",
  "gene_symbol": "WNT8A"
}